{
  "term_id": "UNKNOWN:0003",
  "gene_symbol": "PLD5",
  "gene_name": "Inactive phospholipase D5",
  "gene": "UniProtKB:Q8N7P1",
  "term_label": "Unknown cellular component"
}